negative regulation of skeletal muscle cell differentiation [GO:2001015] (biological process) Subtypes: negative regulation of satellite cell differentiation [GO:1902725], GO:1902810 Definition: Any process that stops, prevents or reduces the frequency, rate or extent of skeletal muscle cell differentiation. Relationships: is a type of GO:0045596; is a type of GO:2001014; negatively regulates skeletal muscle cell differentiation [GO:0035914] Sources: GOC:obol